stomatal complex patterning [GO:0010375] (biological process) Definition: The regionalization process of establishing the non-random spatial arrangement of stomatal complex on the surface of a leaf. The stomatal complex is the stomatal guard cells and their associated epidermal cells. Relationships: is_a regionalization [GO:0003002] References: PMID:17259259 Regulation: regulated by GO:2000037